carbon-oxygen lyase activity, acting on polysaccharides [GO:0016837] (molecular function) Relationships: is a type of carbon-oxygen lyase activity [GO:0016835] Definition: Catalysis of the cleavage of a carbon-oxygen bond by the elimination of an alcohol from a polysaccharide. Subtypes: peptidoglycan lytic transglycosylase activity [GO:0008933], GO:0015021, GO:0030340, chondroitin AC lyase activity [GO:0030341], pectate lyase activity [GO:0030570], glucuronan lyase activity [GO:0033994], GO:0033995, levan fructotransferase (DFA-IV-forming) activity [GO:0033996], inulin fructotransferase (DFA-I-forming) activity [GO:0033997], inulin fructotransferase (DFA-III-forming) activity [GO:0033998], GO:0033999, GO:0034000, chondroitin-sulfate-ABC exolyase activity [GO:0034001], poly(beta-D-mannuronate) lyase activity [GO:0045135], rhamnogalacturonan alpha-L-rhamnopyranosyl-(1->4)-alpha-D-galactopyranosyluronide lyase activity [GO:0046576], exo-(1,4)-alpha-D-glucan lyase activity [GO:0047457], oligogalacturonide lyase activity [GO:0047487], heparin lyase activity [GO:0047488], pectate disaccharide-lyase activity [GO:0047489], pectin lyase activity [GO:0047490], poly(alpha-L-guluronate) lyase activity [GO:0047491], GO:0047492, gellan lyase activity [GO:0052762], GO:0052763, exo-oligoalginate lyase activity [GO:0052764], acharan sulfate lyase activity [GO:0052809], rhamnogalacturonan endolyase activity [GO:0102210] Sources: EC:4.2.2.-